{
  "gene": "UniProtKB:P86478",
  "term_label": "Unknown cellular component",
  "gene_name": "Proline-rich protein 20E",
  "term_id": "UNKNOWN:0003",
  "gene_symbol": "PRR20E"
}